{
  "term_label": "negative regulation of inflammatory response",
  "gene_name": "NLR family CARD domain-containing protein 3",
  "gene": "UniProtKB:Q7RTR2",
  "gene_symbol": "NLRC3",
  "term_id": "GO:0050728"
}